{
  "term_id": "UNKNOWN:0001",
  "gene_symbol": "SOWAHB",
  "term_label": "Unknown molecular function",
  "gene": "UniProtKB:A6NEL2",
  "gene_name": "Ankyrin repeat domain-containing protein SOWAHB"
}